{
  "term_id": "UNKNOWN:0001",
  "gene_name": "Tumor necrosis factor receptor superfamily member 14",
  "gene_symbol": "TNFRSF14",
  "gene": "UniProtKB:Q92956",
  "term_label": "Unknown molecular function"
}